{
  "gene_symbol": "SFTPC",
  "term_label": "Unknown molecular function",
  "gene": "UniProtKB:P11686",
  "gene_name": "Pulmonary surfactant-associated protein C",
  "term_id": "UNKNOWN:0001"
}